{
  "gene": "UniProtKB:Q9Y4L1",
  "term_id": "GO:0000774",
  "gene_symbol": "HYOU1",
  "term_label": "adenyl-nucleotide exchange factor activity",
  "gene_name": "Hypoxia up-regulated protein 1"
}